{
  "gene": "UniProtKB:Q9Y3M2",
  "gene_name": "Protein chibby homolog 1",
  "term_id": "GO:0005634",
  "term_label": "nucleus",
  "gene_symbol": "CBY1"
}